regulation of regulatory T cell differentiation [GO:0045589] (biological process) Subtypes: regulation of CD4-positive, CD25-positive, alpha-beta regulatory T cell differentiation [GO:0032829], negative regulation of regulatory T cell differentiation [GO:0045590], positive regulation of regulatory T cell differentiation [GO:0045591] Sources: ISBN:0781735149 Note: Note that immunologists typically use the word 'development' to refer to cells of B or T cell lineages undergoing the process that GO describes as 'cell differentiation'. Definition: Any process that modulates the frequency, rate or extent of differentiation of regulatory T cells. Also known as: regulation of regulatory T lymphocyte differentiation, regulation of regulatory T-cell differentiation, regulation of regulatory T-lymphocyte differentiation, regulation of suppressor T cell differentiation, regulation of suppressor T lymphocyte differentiation, regulation of suppressor T-cell differentiation, regulation of suppressor T-lymphocyte differentiation, regulation of regulatory T cell development Relationships: is a type of regulation of T cell differentiation [GO:0045580]; regulates GO:0045066